{
  "gene": "UniProtKB:P07333",
  "term_label": "CSF1-CSF1R complex",
  "gene_name": "Macrophage colony-stimulating factor 1 receptor",
  "term_id": "GO:1990682",
  "gene_symbol": "CSF1R"
}